{
  "term_label": "Ras protein signal transduction",
  "gene_name": "GTPase KRas",
  "gene_symbol": "KRAS",
  "term_id": "GO:0007265",
  "gene": "UniProtKB:P01116"
}